farnesal dehydrogenase (NAD+) activity [GO:0120553] (MF) Relationships: is a type of GO:0004029 Definition: Catalysis of the reaction: (2E,6E)-farnesal + NAD+ + H2O = (2E,6E)-farnesoate + NADH + 2 H+. References: PMID:23639754 Sources: RHEA:24216